{
  "gene_name": "Heterogeneous nuclear ribonucleoprotein R",
  "term_label": "ribonucleoprotein complex",
  "term_id": "GO:1990904",
  "gene": "UniProtKB:O43390",
  "gene_symbol": "HNRNPR"
}